{
  "gene_name": "Nuclear envelope phosphatase-regulatory subunit 1",
  "term_id": "UNKNOWN:0001",
  "gene": "UniProtKB:Q8N9A8",
  "term_label": "Unknown molecular function",
  "gene_symbol": "CNEP1R1"
}